regulation of urine volume [GO:0035809] (biological process) Subtypes: GO:0035810, negative regulation of urine volume [GO:0035811] Definition: Any process that modulates the amount of urine excreted from the body over a unit of time. Also known as: regulation of urinary volume, regulation of urine flow Sources: GOC:mtg_25march11, GOC:yaf Relationships: is a type of renal system process [GO:0003014]; is_a regulation of body fluid levels [GO:0050878]